{
  "gene_symbol": "GABBR2",
  "gene": "UniProtKB:O75899",
  "term_id": "GO:0004888",
  "gene_name": "Gamma-aminobutyric acid type B receptor subunit 2",
  "term_label": "transmembrane signaling receptor activity"
}